smooth muscle hypertrophy [GO:0014895] (biological process) Sources: GOC:mtg_muscle Definition: The enlargement or overgrowth of all or part of an organ due to an increase in size of its smooth muscle cells without cell division. Physiological hypertrophy is a normal process during development, and can also occur in mature structures on demand. In the uterus, smooth muscle cells undergo hypertrophy during pregnancy. Relationships: is a type of smooth muscle adaptation [GO:0014805]; is a type of GO:0014896 Regulation: regulated by regulation of smooth muscle hypertrophy [GO:1905147]; negatively regulated by negative regulation of smooth muscle hypertrophy [GO:1905148]; positively regulated by positive regulation of smooth muscle hypertrophy [GO:1905149]